{
  "term_label": "GPI anchor biosynthetic process",
  "gene_name": "Phosphatidylinositol N-acetylglucosaminyltransferase subunit A",
  "gene_symbol": "PIGA",
  "gene": "UniProtKB:P37287",
  "term_id": "GO:0006506"
}